{
  "gene_name": "Ectonucleotide pyrophosphatase_phosphodiesterase family member 1",
  "term_label": "dinucleotide phosphatase activity",
  "term_id": "GO:0004551",
  "gene_symbol": "ENPP1",
  "gene": "UniProtKB:P22413"
}